{
  "gene_symbol": "C1R",
  "term_label": "serine-type endopeptidase activity",
  "gene_name": "Complement C1r subcomponent",
  "gene": "UniProtKB:P00736",
  "term_id": "GO:0004252"
}